cytosine/cytosine mispair binding [GO:0035486] (molecular function) Definition: Binding to a double-stranded DNA region containing a C/C mispair. Relationships: is a type of mismatched DNA binding [GO:0030983] Sources: GOC:bf, GOC:jh Also known as: C/C mispair binding